sarcosine dehydrogenase activity [GO:0008480] (molecular function) Definition: Catalysis of the reaction: sarcosine + H2O + electron-transfer flavoprotein = glycine + formaldehyde + reduced electron-transfer flavoprotein. Note: Note that this was EC:1.5.99.1. Also known as: monomethylglycine dehydrogenase activity, sarcosine N-demethylase activity, sarcosine:(acceptor) oxidoreductase (demethylating), sarcosine:acceptor oxidoreductase (demethylating) Relationships: is a type of oxidoreductase activity, acting on the CH-NH group of donors, flavin as acceptor [GO:0046997] Sources: EC:1.5.8.3, RHEA:19793